acetylcholine catabolic process [GO:0006581] (biological process) Subtypes: GO:0001507 Definition: The chemical reactions and pathways resulting in the breakdown of acetylcholine, the acetic acid ester of the organic base choline. Relationships: is a type of acetylcholine metabolic process [GO:0008291]; is a type of catabolic process [GO:0009056] Sources: GOC:jl, ISBN:0192800752 Also known as: acetylcholine breakdown, acetylcholine catabolism, acetylcholine degradation